{
  "term_label": "TRAPP complex",
  "term_id": "GO:0030008",
  "gene": "UniProtKB:Q9Y296",
  "gene_symbol": "TRAPPC4",
  "gene_name": "Trafficking protein particle complex subunit 4"
}